membrane repolarization during action potential [GO:0086011] (biological process) Regulation: regulated by regulation of membrane repolarization during action potential [GO:0098903] Relationships: is a type of membrane repolarization [GO:0086009]; is part of action potential [GO:0001508] Definition: The process in which ions are transported across a membrane such that the membrane potential changes in the direction from the positive membrane potential at the peak of the action potential towards the negative resting potential. Subtypes: membrane repolarization during cardiac muscle cell action potential [GO:0086013] Sources: GOC:BHF, GOC:mtg_cardiac_conduct_nov11